{
  "gene": "UniProtKB:Q7L8C5",
  "term_label": "synaptic vesicle membrane",
  "gene_name": "Synaptotagmin-13",
  "gene_symbol": "SYT13",
  "term_id": "GO:0030672"
}